{
  "gene_symbol": "RAB7A",
  "gene_name": "Ras-related protein Rab-7a",
  "term_id": "GO:0045335",
  "gene": "UniProtKB:P51149",
  "term_label": "phagocytic vesicle"
}